{
  "gene_name": "Homeobox protein CDX-4",
  "term_id": "GO:0006357",
  "term_label": "regulation of transcription by RNA polymerase II",
  "gene_symbol": "CDX4",
  "gene": "UniProtKB:O14627"
}